{
  "term_id": "UNKNOWN:0002",
  "gene": "UniProtKB:Q6P2H3",
  "gene_name": "Centrosomal protein of 85 kDa",
  "gene_symbol": "CEP85",
  "term_label": "Unknown biological process"
}